{
  "gene_name": "Protein CD300H",
  "term_label": "signal transduction",
  "gene": "UniProtKB:A0A0K2S4Q6",
  "gene_symbol": "CD300H",
  "term_id": "GO:0007165"
}